{
  "gene_symbol": "CELF1",
  "gene_name": "CUGBP Elav-like family member 1",
  "term_id": "GO:0003730",
  "gene": "UniProtKB:Q92879",
  "term_label": "mRNA 3'-UTR binding"
}